modification of synaptic structure, modulating synaptic transmission [GO:0099564] (biological process) Relationships: is a type of modification of synaptic structure [GO:0099563]; regulates chemical synaptic transmission [GO:0007268] Sources: GOC:dos Note: Note that this term was created for the SynGO project, and will be obsoleted when the SynGO annotations are made in Noctua. Definition: Any process that modulates synaptic transmission via modification of the structure of the synapse.